epi-cedrol synthase activity [GO:0052682] (MF) Sources: RHEA:26115 Definition: Catalysis of the reaction: 2-trans,6-trans-farnesyl diphosphate + H2O = epi-cedrol + diphosphate. Relationships: is a type of carbon-oxygen lyase activity, acting on phosphates [GO:0016838] Also known as: (2E,6E)-farnesyl-diphosphate diphosphate-lyase (8-epi-cedrol-forming) activity, 8-epicedrol synthase activity, epicedrol synthase activity